{
  "gene_symbol": "BRICD5",
  "gene": "UniProtKB:Q6PL45",
  "term_id": "GO:0005615",
  "gene_name": "BRICHOS domain-containing protein 5",
  "term_label": "extracellular space"
}